{
  "gene": "UniProtKB:Q86VZ1",
  "gene_name": "P2Y purinoceptor 8",
  "term_label": "G protein-coupled receptor signaling pathway",
  "gene_symbol": "P2RY8",
  "term_id": "GO:0007186"
}